{
  "gene_symbol": "RAB22A",
  "term_label": "GTPase activity",
  "gene_name": "Ras-related protein Rab-22A",
  "gene": "UniProtKB:Q9UL26",
  "term_id": "GO:0003924"
}